acyltransferase activity, acyl groups converted into alkyl on transfer [GO:0046912] (molecular function) Definition: Catalysis of the transfer of an acyl group from one compound (donor) to another (acceptor), with the acyl group being converted into alkyl on transfer. Sources: GOC:jl Also known as: acyltransferase, acyl groups converted into alkyl on transfer, transferase activity, transferring acyl groups, acyl groups converted into alkyl on transfer Relationships: is a type of GO:0016746 Subtypes: GO:0003852, ATP citrate synthase activity [GO:0003878], homocitrate synthase activity [GO:0004410], hydroxymethylglutaryl-CoA synthase activity [GO:0004421], malate synthase activity [GO:0004474], methylthioalkylmalate synthase activity [GO:0010177], 2-hydroxyglutarate synthase activity [GO:0019142], citrate synthase activity [GO:0036440], 2-ethylmalate synthase activity [GO:0050438], GO:0050440, 3-ethylmalate synthase activity [GO:0050441], 3-propylmalate synthase activity [GO:0050442], GO:0050457, decylhomocitrate synthase activity [GO:0050458], sulfoacetaldehyde acetyltransferase activity [GO:0050487]